organelle membrane contact site [GO:0044232] (CC) Definition: A zone of apposition between the membranes of an organelle with another membrane, either another membrane of the same organelle, a membrane of another organelle, or the plasma membrane. Membrane contact sites (MCSs) are structured by bridging complexes. They are specialized for communication, including the efficient traffic of small molecules such as Ca2+ ions and lipids, as well as enzyme-substrate interactions. Relationships: is a type of cellular anatomical structure [GO:0110165]; is part of organelle [GO:0043226] Subtypes: mitochondria-associated endoplasmic reticulum membrane contact site [GO:0044233], mitochondrial crista junction [GO:0044284], GO:0044289, GO:0071561, GO:0098853, GO:0120095, endoplasmic reticulum-plasma membrane contact site [GO:0140268], endoplasmic reticulum-endosome membrane contact site [GO:0140284], peroxisomal-mitochondrial contact site [GO:0160189], GO:0160258, vacuole-mitochondrion membrane contact site [GO:1990816] Also known as: MCS, inter-organelle junction, interorganelle junction References: PMID:16806880 Sources: GOC:jl